positive regulation of luteinizing hormone secretion [GO:0033686] (biological process) Definition: Any process that activates or increases the frequency, rate or extent of the regulated release of luteinizing hormone. Sources: GOC:mah Also known as: up regulation of luteinizing hormone secretion, up-regulation of luteinizing hormone secretion, upregulation of luteinizing hormone secretion, activation of luteinizing hormone secretion, stimulation of luteinizing hormone secretion Relationships: is a type of positive regulation of gonadotropin secretion [GO:0032278]; is_a regulation of luteinizing hormone secretion [GO:0033684]; positively regulates luteinizing hormone secretion [GO:0032275]